{
  "gene": "UniProtKB:Q96KV7",
  "gene_symbol": "WDR90",
  "gene_name": "WD repeat-containing protein 90",
  "term_id": "UNKNOWN:0001",
  "term_label": "Unknown molecular function"
}